{
  "gene_name": "FAS-associated death domain protein",
  "term_label": "death receptor binding",
  "term_id": "GO:0005123",
  "gene": "UniProtKB:Q13158",
  "gene_symbol": "FADD"
}